{
  "term_id": "UNKNOWN:0003",
  "gene": "UniProtKB:Q9NUB4",
  "gene_symbol": "C20orf141",
  "gene_name": "Uncharacterized protein C20orf141",
  "term_label": "Unknown cellular component"
}